{
  "term_label": "nucleosomal DNA binding",
  "term_id": "GO:0031492",
  "gene": "UniProtKB:Q71DI3",
  "gene_symbol": "H3C13",
  "gene_name": "Histone H3.2"
}